{
  "term_id": "GO:1904263",
  "gene": "UniProtKB:O43504",
  "gene_symbol": "LAMTOR5",
  "gene_name": "Ragulator complex protein LAMTOR5",
  "term_label": "positive regulation of TORC1 signaling"
}